{
  "gene_name": "Ras-related protein Rab-36",
  "term_label": "GTP binding",
  "gene_symbol": "RAB36",
  "gene": "UniProtKB:O95755",
  "term_id": "GO:0005525"
}